{
  "term_id": "GO:0006271",
  "gene_symbol": "MCM4",
  "gene": "UniProtKB:P33991",
  "gene_name": "DNA replication licensing factor MCM4",
  "term_label": "DNA strand elongation involved in DNA replication"
}